negative regulation of nuclear receptor-mediated glucocorticoid signaling pathway [GO:2000323] (biological process) Relationships: is a type of GO:0033144; is a type of regulation of nuclear receptor-mediated glucocorticoid signaling pathway [GO:2000322]; negatively regulates nuclear receptor-mediated glucocorticoid signaling pathway [GO:0042921] Definition: Any process that stops, prevents or reduces the frequency, rate or extent of nuclear receptor-mediated glucocorticoid signaling pathway. Also known as: negative regulation of glucocorticoid receptor signaling pathway, negative regulation of glucocorticoid receptor signalling pathway Sources: GOC:BHF